{
  "term_label": "chromosome passenger complex",
  "gene_name": "Aurora kinase C",
  "gene_symbol": "AURKC",
  "gene": "UniProtKB:Q9UQB9",
  "term_id": "GO:0032133"
}